{
  "gene_name": "Protein KTI12 homolog",
  "gene": "UniProtKB:Q96EK9",
  "gene_symbol": "KTI12",
  "term_label": "Unknown cellular component",
  "term_id": "UNKNOWN:0003"
}